{
  "term_label": "midbody",
  "term_id": "GO:0030496",
  "gene_symbol": "MTCL1",
  "gene_name": "Microtubule cross-linking factor 1",
  "gene": "UniProtKB:Q9Y4B5"
}